{
  "gene_symbol": "GOLGA2P5",
  "gene": "UniProtKB:Q9HBQ8",
  "term_id": "UNKNOWN:0001",
  "term_label": "Unknown molecular function",
  "gene_name": "Putative golgin subfamily A member 2B"
}